{
  "gene": "UniProtKB:P57103",
  "term_id": "GO:0098794",
  "term_label": "postsynapse",
  "gene_symbol": "SLC8A3",
  "gene_name": "Sodium_calcium exchanger 3"
}